{
  "gene": "UniProtKB:Q9HAU4",
  "term_id": "GO:0005737",
  "gene_symbol": "SMURF2",
  "term_label": "cytoplasm",
  "gene_name": "E3 ubiquitin-protein ligase SMURF2"
}